{
  "gene_symbol": "SULT1A1",
  "gene": "UniProtKB:P50225",
  "gene_name": "Sulfotransferase 1A1",
  "term_label": "sulfation",
  "term_id": "GO:0051923"
}